positive regulation of vacuole fusion, non-autophagic [GO:0061191] (biological process) Sources: GOC:dph Definition: Any process that increases the frequency, rate or extent of the fusion of two vacuole membranes to form a single vacuole. Relationships: is a type of GO:0032889; is a type of positive regulation of vacuole organization [GO:0044090]; positively regulates GO:0042144